{
  "gene_name": "Mothers against decapentaplegic homolog 7",
  "term_label": "heteromeric SMAD protein complex",
  "term_id": "GO:0071144",
  "gene": "UniProtKB:O15105",
  "gene_symbol": "SMAD7"
}